{
  "gene_name": "Synapsin-3",
  "gene": "UniProtKB:O14994",
  "term_label": "synapse organization",
  "term_id": "GO:0050808",
  "gene_symbol": "SYN3"
}